{
  "gene_symbol": "RBMS1",
  "gene_name": "RNA-binding motif, single-stranded-interacting protein 1",
  "gene": "UniProtKB:P29558",
  "term_label": "ribonucleoprotein complex",
  "term_id": "GO:1990904"
}